{
  "gene": "UniProtKB:Q03164",
  "gene_symbol": "KMT2A",
  "term_id": "GO:0045893",
  "term_label": "positive regulation of DNA-templated transcription",
  "gene_name": "Histone-lysine N-methyltransferase 2A"
}